{
  "gene": "UniProtKB:Q9BY50",
  "gene_name": "Signal peptidase complex catalytic subunit SEC11C",
  "term_label": "signal peptidase complex",
  "gene_symbol": "SEC11C",
  "term_id": "GO:0005787"
}